positive regulation of megakaryocyte differentiation [GO:0045654] (biological process) Also known as: up regulation of megakaryocyte differentiation, up-regulation of megakaryocyte differentiation, upregulation of megakaryocyte differentiation, activation of megakaryocyte differentiation, stimulation of megakaryocyte differentiation Sources: GOC:go_curators Relationships: is a type of positive regulation of myeloid cell differentiation [GO:0045639]; is_a regulation of megakaryocyte differentiation [GO:0045652]; positively regulates megakaryocyte differentiation [GO:0030219] Definition: Any process that activates or increases the frequency, rate or extent of megakaryocyte differentiation.